Golgi vesicle uncoating [GO:0048212] (biological process) References: PMID:10219233 Sources: GOC:jid, ISBN:0716731363 Definition: The process in which Golgi vesicle coat proteins are depolymerized, and released for reuse. Also known as: Golgi vesicle coat depolymerization, Golgi vesicle coat protein depolymerization, Golgi-derived vesicle uncoating, dictyosome vesicle coat depolymerization Relationships: is a type of vesicle uncoating [GO:0072319]; is part of Golgi vesicle transport [GO:0048193]